{
  "term_label": "regulation of transcription by RNA polymerase II",
  "gene": "UniProtKB:P15822",
  "gene_symbol": "HIVEP1",
  "term_id": "GO:0006357",
  "gene_name": "Zinc finger protein 40"
}